{
  "gene_name": "Serine_threonine-protein phosphatase 2B catalytic subunit gamma isoform",
  "gene": "UniProtKB:P48454",
  "gene_symbol": "PPP3CC",
  "term_label": "calcineurin-mediated signaling",
  "term_id": "GO:0097720"
}